MyD88-dependent toll-like receptor signaling pathway [GO:0002755] (biological process) Regulation: regulated by regulation of MyD88-dependent toll-like receptor signaling pathway [GO:0034124]; negatively regulated by negative regulation of MyD88-dependent toll-like receptor signaling pathway [GO:0034125]; positively regulated by positive regulation of MyD88-dependent toll-like receptor signaling pathway [GO:0034126] Also known as: MyD88-dependent TLR signaling pathway, MyD88-dependent toll-like receptor signalling pathway References: PMID:12467241, PMID:12524386, PMID:12855817, PMID:15585605, PMID:15728447 Sources: GOC:add, ISBN:0781735149 Relationships: is a type of toll-like receptor signaling pathway [GO:0002224] Definition: A toll-like receptor signaling pathway in which the MyD88 adaptor molecule mediates transduction of the signal. Toll-like receptors directly bind pattern motifs from a variety of microbial sources to initiate an innate immune response. Subtypes: MyD88-dependent toll-like receptor 4 signaling pathway [GO:0035660], MyD88-dependent toll-like receptor 2 signaling pathway [GO:0035661]